methaneselenol methyltransferase activity [GO:0098613] (molecular function) References: PMID:14705, PMID:17988700, PMID:4380351 Definition: Catalysis of the reaction: S-adenosyl-L-methionine + methaneselenol = S-adenosyl-L-homocysteine + dimethyl selenide. Relationships: is_a GO:0008168